{
  "gene_symbol": "PGA3",
  "term_label": "aspartic-type endopeptidase activity",
  "gene_name": "Pepsin A-3",
  "term_id": "GO:0004190",
  "gene": "UniProtKB:P0DJD8"
}